{
  "gene_symbol": "CCND1",
  "term_id": "GO:1900087",
  "term_label": "positive regulation of G1/S transition of mitotic cell cycle",
  "gene_name": "G1_S-specific cyclin-D1",
  "gene": "UniProtKB:P24385"
}